{
  "gene_name": "Exosome complex component RRP43",
  "gene_symbol": "EXOSC8",
  "gene": "UniProtKB:Q96B26",
  "term_label": "nuclear mRNA surveillance",
  "term_id": "GO:0071028"
}